{
  "gene": "UniProtKB:Q8IYX4",
  "gene_symbol": "DND1",
  "term_label": "cytoplasm",
  "term_id": "GO:0005737",
  "gene_name": "Dead end protein homolog 1"
}